{
  "gene_symbol": "UBE2QL1",
  "term_id": "GO:0061631",
  "gene_name": "Ubiquitin-conjugating enzyme E2Q-like protein 1",
  "gene": "UniProtKB:A1L167",
  "term_label": "ubiquitin conjugating enzyme activity"
}